{
  "term_id": "GO:0043123",
  "gene": "UniProtKB:Q12933",
  "gene_symbol": "TRAF2",
  "term_label": "positive regulation of canonical NF-kappaB signal transduction",
  "gene_name": "TNF receptor-associated factor 2"
}